pollen hydration [GO:0009859] (biological process) Relationships: is a type of GO:0006833; is part of pollen-pistil interaction [GO:0009875] Sources: GOC:lr Definition: The process in which water is taken up by pollen.